{
  "gene": "UniProtKB:P29973",
  "gene_symbol": "CNGA1",
  "term_id": "GO:0005222",
  "term_label": "intracellularly cAMP-activated cation channel activity",
  "gene_name": "cGMP-gated cation channel alpha-1"
}